{
  "gene": "UniProtKB:Q2M385",
  "term_id": "UNKNOWN:0003",
  "term_label": "Unknown cellular component",
  "gene_symbol": "MPEG1",
  "gene_name": "Macrophage-expressed gene 1 protein"
}